{
  "term_id": "UNKNOWN:0001",
  "gene_name": "Protein phosphatase 1 regulatory subunit 42",
  "term_label": "Unknown molecular function",
  "gene_symbol": "PPP1R42",
  "gene": "UniProtKB:Q7Z4L9"
}